{
  "gene_symbol": "CARNMT1",
  "gene_name": "Carnosine N-methyltransferase",
  "term_id": "GO:0030735",
  "gene": "UniProtKB:Q8N4J0",
  "term_label": "carnosine N-methyltransferase activity"
}